high-affinity fructose transmembrane transporter activity [GO:0061486] (molecular function) References: PMID:10735857 Sources: GOC:dph Also known as: high affinity fructose transmembrane transporter activity Relationships: is_a GO:0005353 Definition: Enables the transfer of fructose from one side of a membrane to the other. In high-affinity transport the transporter is able to bind the solute even if it is only present at very low concentrations.